{
  "term_label": "GTPase activator activity",
  "gene_name": "TBC1 domain family member 1",
  "term_id": "GO:0005096",
  "gene_symbol": "TBC1D1",
  "gene": "UniProtKB:Q86TI0"
}